{
  "gene_name": "Myelin regulatory factor",
  "gene_symbol": "MYRF",
  "term_label": "sequence-specific DNA binding",
  "term_id": "GO:0043565",
  "gene": "UniProtKB:Q9Y2G1"
}